{
  "gene_symbol": "SORT1",
  "term_id": "GO:0010465",
  "term_label": "nerve growth factor receptor activity",
  "gene": "UniProtKB:Q99523",
  "gene_name": "Sortilin"
}